chemorepulsion involved in precerebellar neuron migration [GO:0021950] (biological process) Definition: The creation and reception of signals that repel a precerebellar neuron as a component of the process of tangential migration. References: PMID:15157725 Sources: GOC:cls, GOC:dgh, GOC:dph, GOC:jid, GO_REF:0000021 Also known as: negative chemotaxis involved in precerebellar neuron migration Relationships: is a type of negative chemotaxis [GO:0050919]; is part of brainstem precerebellar neuron precursor migration [GO:0021949]